{
  "gene_symbol": "TBC1D24",
  "gene_name": "TBC1 domain family member 24",
  "term_id": "UNKNOWN:0002",
  "term_label": "Unknown biological process",
  "gene": "UniProtKB:Q9ULP9"
}